protein localization to CENP-A containing chromatin [GO:0061644] (biological process) Sources: GOC:dph, GOC:vw Relationships: is_a protein localization to chromatin [GO:0071168]; is a type of protein localization to chromosome, centromeric region [GO:0071459] Definition: Any process in which a protein is transported to, or maintained at, CENP-A containing chromatin.